{
  "gene_symbol": "PXDN",
  "term_label": "peroxidase activity",
  "gene_name": "Peroxidasin homolog",
  "term_id": "GO:0004601",
  "gene": "UniProtKB:Q92626"
}